anther morphogenesis [GO:0048654] (BP) Definition: The process in which the anatomical structures of the anther are generated and organized. Sources: GOC:jid, GOC:sm Relationships: is a type of floral organ morphogenesis [GO:0048444]; is part of GO:0048448; is part of GO:0048653